G protein-coupled receptor kinase activity [GO:0004703] (molecular function) Definition: Catalysis of the reaction: ATP + G protein-coupled receptor = ADP + G protein-coupled receptor phosphate. Also known as: G protein coupled receptor phosphorylating protein kinase activity, G-protein-coupled receptor phosphorylating protein kinase activity, GPCR phosphorylating protein kinase activity, ATP:G-protein-coupled receptor phosphotransferase activity, G-protein coupled receptor kinase activity, GPCR kinase activity, GPCRK, GRK4, GRK5, GRK6, STK16 Sources: GOC:dph Subtypes: GO:0050254 Relationships: is a type of protein serine/threonine kinase activity [GO:0004674]